{
  "gene_name": "Phospholipid hydroperoxide glutathione peroxidase",
  "gene": "UniProtKB:P36969",
  "term_id": "GO:0005739",
  "gene_symbol": "GPX4",
  "term_label": "mitochondrion"
}